cyclin B3-CDK2 complex [GO:0097127] (cellular component) References: PMID:15935619 Sources: GOC:so Relationships: is a type of cyclin-dependent protein kinase holoenzyme complex [GO:0000307] Definition: A protein complex consisting of cyclin B3 and cyclin-dependent kinase 2 (CDK2). Cyclins are characterized by periodicity in protein abundance throughout the cell cycle. Cyclin-dependent kinases represent a family of serine/threonine protein kinases that become active upon binding to a cyclin regulatory partner.